negative regulation of syringal lignin catabolic process [GO:1901470] (biological process) Definition: Any process that stops, prevents or reduces the frequency, rate or extent of syringal lignin catabolic process. Sources: GOC:TermGenie, GOC:mengo_curators Also known as: down regulation of S-lignin catabolic process, down regulation of syringal lignin breakdown, down regulation of syringal lignin catabolic process, down regulation of syringal lignin catabolism, down regulation of syringal lignin degradation, down-regulation of S-lignin catabolic process, down-regulation of syringal lignin breakdown, down-regulation of syringal lignin catabolic process, down-regulation of syringal lignin catabolism, down-regulation of syringal lignin degradation, downregulation of S-lignin catabolic process, downregulation of syringal lignin breakdown, downregulation of syringal lignin catabolic process, downregulation of syringal lignin catabolism, downregulation of syringal lignin degradation, inhibition of S-lignin catabolic process, inhibition of syringal lignin breakdown, inhibition of syringal lignin catabolism, inhibition of syringal lignin degradation, negative regulation of S-lignin catabolic process, negative regulation of syringal lignin breakdown, negative regulation of syringal lignin catabolism, negative regulation of syringal lignin degradation, inhibition of syringal lignin catabolic process Relationships: is a type of negative regulation of catabolic process [GO:0009895]; is a type of regulation of syringal lignin catabolic process [GO:1901469]; negatively regulates syringal lignin catabolic process [GO:1901065]